{
  "gene": "UniProtKB:Q14344",
  "term_label": "G-protein beta/gamma-subunit complex binding",
  "term_id": "GO:0031683",
  "gene_symbol": "GNA13",
  "gene_name": "Guanine nucleotide-binding protein subunit alpha-13"
}